{
  "term_label": "DNA synthesis involved in DNA repair",
  "gene_name": "DNA polymerase alpha catalytic subunit",
  "term_id": "GO:0000731",
  "gene_symbol": "POLA1",
  "gene": "UniProtKB:P09884"
}